salicylate 5-hydroxylase (NADH) activity [GO:0034785] (molecular function) Definition: Catalysis of the reaction: salicylate + NADH + O2 + H+ = 2,5-dihydroxybenzoate + NAD+ + H2O. Sources: RHEA:35307 Relationships: is a type of oxidoreductase activity, acting on paired donors, with incorporation or reduction of molecular oxygen, NAD(P)H as one donor, and incorporation of one atom of oxygen [GO:0016709]